{
  "gene": "UniProtKB:P51884",
  "term_label": "collagen binding",
  "gene_name": "Lumican",
  "term_id": "GO:0005518",
  "gene_symbol": "LUM"
}